guanylate cyclase regulator activity [GO:0030249] (molecular function) Definition: Modulates the activity of guanylate cyclase. Relationships: is_a cyclase regulator activity [GO:0010851]; regulates GO:0004383 Subtypes: guanylate cyclase activator activity [GO:0030250], guanylate cyclase inhibitor activity [GO:0030251] Sources: GOC:mah